recycling endosome to Golgi transport [GO:0071955] (biological process) Sources: GOC:lb Relationships: is a type of retrograde transport, endosome to Golgi [GO:0042147]; is a type of Golgi vesicle transport [GO:0048193] Definition: The directed movement of substances from recycling endosomes to the Golgi.